{
  "term_label": "nucleus",
  "gene": "UniProtKB:Q7Z6K1",
  "term_id": "GO:0005634",
  "gene_symbol": "THAP5",
  "gene_name": "THAP domain-containing protein 5"
}